regulation of telomeric loop disassembly [GO:1904533] (biological process) Subtypes: negative regulation of telomeric loop disassembly [GO:1904534], GO:1904535, regulation of telomeric D-loop disassembly [GO:1905838] Definition: Any process that modulates the frequency, rate or extent of telomeric loop disassembly. Relationships: is a type of GO:0032204; RO_0002211 telomeric loop disassembly [GO:0090657] Also known as: regulation of T loop disassembly References: PMID:22579284 Sources: GOC:BHF, GOC:BHF_telomere, GOC:TermGenie, GOC:nc, GO_REF:0000058